specification of segmental identity, maxillary segment [GO:0007382] (biological process) Sources: ISBN:0878932437 Definition: The specification of the characteristic structures of the maxillary segment following establishment of segment boundaries. Identity is considered to be the aggregate of characteristics by which a structure is recognized. Relationships: is a type of specification of segmental identity, head [GO:0007380]; is part of posterior head segmentation [GO:0035289] Note: See also the fly_anatomy.ontology term 'maxillary segment ; FBbt:00000013'.